{
  "term_id": "GO:0044774",
  "term_label": "mitotic DNA integrity checkpoint signaling",
  "gene": "UniProtKB:Q53H47",
  "gene_symbol": "SETMAR",
  "gene_name": "Histone-lysine N-methyltransferase SETMAR"
}